{
  "gene_symbol": "ALX3",
  "gene": "UniProtKB:O95076",
  "gene_name": "Homeobox protein aristaless-like 3",
  "term_id": "GO:0000977",
  "term_label": "RNA polymerase II transcription regulatory region sequence-specific DNA binding"
}